{
  "gene_name": "Probable ATP-dependent RNA helicase DDX31",
  "term_id": "GO:0042254",
  "gene": "UniProtKB:Q9H8H2",
  "gene_symbol": "DDX31",
  "term_label": "ribosome biogenesis"
}